{
  "gene_symbol": "KIF6",
  "term_id": "GO:0003777",
  "gene": "UniProtKB:Q6ZMV9",
  "gene_name": "Kinesin-like protein KIF6",
  "term_label": "microtubule motor activity"
}